glutamate receptor binding [GO:0035254] (MF) Sources: GOC:bf Relationships: is a type of GO:0005102 Subtypes: GO:0035255, G protein-coupled glutamate receptor binding [GO:0035256] Definition: Binding to a glutamate receptor.